{
  "gene_name": "Catenin delta-1",
  "gene": "UniProtKB:O60716",
  "term_label": "cytoplasm",
  "gene_symbol": "CTNND1",
  "term_id": "GO:0005737"
}